{
  "term_label": "Unknown biological process",
  "gene": "UniProtKB:Q9BVV2",
  "gene_symbol": "FNDC11",
  "term_id": "UNKNOWN:0002",
  "gene_name": "Fibronectin type III domain-containing protein 11"
}